{
  "term_label": "translation elongation factor activity",
  "term_id": "GO:0003746",
  "gene_symbol": "TSFM",
  "gene": "UniProtKB:P43897",
  "gene_name": "Elongation factor Ts, mitochondrial"
}